{
  "gene": "UniProtKB:O14965",
  "term_label": "Unknown molecular function",
  "gene_name": "Aurora kinase A",
  "term_id": "UNKNOWN:0001",
  "gene_symbol": "AURKA"
}